multi-organism reproductive process [GO:0044703] (biological process) Subtypes: insemination [GO:0007320], GO:0007565, GO:0007567, mating [GO:0007618], GO:0046692 Definition: A biological process that directly contributes to the process of producing new individuals, involving another organism. Relationships: is a type of reproductive process [GO:0022414] Sources: GOC:jl